conjugation with cellular fusion [GO:0000747] (biological process) Definition: A conjugation process that results in the union of cellular and genetic information from compatible mating types. An example of this process is found in Saccharomyces cerevisiae. Relationships: is a type of sexual reproduction [GO:0019953]; has part cell-cell fusion [GO:0140253] Sources: GOC:elh Also known as: cell fusion, mating Regulation: positively regulated by response to pheromone triggering conjugation with cellular fusion [GO:0000749]; regulated by regulation of conjugation with cellular fusion [GO:0031137]; negatively regulated by GO:0031138; positively regulated by positive regulation of conjugation with cellular fusion [GO:0031139]